{
  "term_label": "miRNA-mediated post-transcriptional gene silencing",
  "term_id": "GO:0035195",
  "gene_symbol": "TNRC6C",
  "gene_name": "Trinucleotide repeat-containing gene 6C protein",
  "gene": "UniProtKB:Q9HCJ0"
}